ATPase-coupled lipid transmembrane transporter activity [GO:0034040] (molecular function) Sources: GOC:BHF, GOC:rl Subtypes: GO:0015432, ABC-type fatty-acyl-CoA transporter activity [GO:0015607], ABC-type sterol transporter activity [GO:0034041] Relationships: is a type of GO:0042626; is a type of lipid transmembrane transporter activity [GO:0170055] Definition: Enables the transfer of a solute or solutes from one side of a membrane to the other according to the reaction: ATP + H2O + lipid(in) = ADP + phosphate + lipid(out). Also known as: lipid-transporting ATPase activity, ATP-dependent lipid transmembrane transporter activity